{
  "gene": "UniProtKB:P60372",
  "term_label": "Unknown biological process",
  "term_id": "UNKNOWN:0002",
  "gene_name": "Keratin-associated protein 10-4",
  "gene_symbol": "KRTAP10-4"
}